{
  "term_label": "nucleus",
  "gene_name": "PPP2R1A-PPP2R2A-interacting phosphatase regulator 1",
  "gene_symbol": "PABIR1",
  "gene": "UniProtKB:Q96E09",
  "term_id": "GO:0005634"
}